{
  "term_label": "Unknown biological process",
  "gene_symbol": "MROH9",
  "gene": "UniProtKB:Q5TGP6",
  "gene_name": "Maestro heat-like repeat-containing protein family member 9",
  "term_id": "UNKNOWN:0002"
}